{
  "term_id": "GO:0008327",
  "gene_symbol": "MBD3L2B",
  "gene_name": "Methyl-CpG-binding domain protein 3-like 2B",
  "gene": "UniProtKB:A0A1B0GVZ6",
  "term_label": "methyl-CpG binding"
}